{
  "term_id": "GO:0005634",
  "term_label": "nucleus",
  "gene_symbol": "FABP2",
  "gene_name": "Fatty acid-binding protein, intestinal",
  "gene": "UniProtKB:P12104"
}